fatty-acyl-CoA transport [GO:0015916] (biological process) Definition: The directed movement of fatty acyl coenzyme A into, out of or within a cell, or between cells, by means of some agent such as a transporter or pore. Fatty acyl coenzyme A is an acyl group linked to 3'-phosphoadenosine-(5')diphospho(4')pantatheine (coenzyme A). Also known as: fatty acyl CoA transport, fatty acyl coenzyme A transport, fatty acyl-CoA transport Relationships: is a type of organic anion transport [GO:0015711]; is a type of GO:0015748; is a type of GO:0015931; is a type of amide transport [GO:0042886]; is a type of thioester transport [GO:1901337] Sources: GOC:ai, ISBN:0198506732 Subtypes: GO:0015876